{
  "term_id": "GO:0043123",
  "term_label": "positive regulation of canonical NF-kappaB signal transduction",
  "gene": "UniProtKB:O14788",
  "gene_name": "Tumor necrosis factor ligand superfamily member 11",
  "gene_symbol": "TNFSF11"
}